{
  "term_label": "Unknown biological process",
  "term_id": "UNKNOWN:0002",
  "gene_symbol": "TMEM221",
  "gene": "UniProtKB:A6NGB7",
  "gene_name": "Transmembrane protein 221"
}